receptor-mediated bacteriophage reversible attachment to host cell [GO:0098001] (biological process) Note: This process was historically defined by the release, by Waring blending or sonication, by dilution and centrifugation, or by filtration and washing, of infective virions from their complexes with cells, thus contrary to what is observed after irreversible adsorption. Relationships: is_a adhesion receptor-mediated virion attachment to host cell [GO:0098671] Also known as: reversible bacteriophage attachment, binding of host cell surface receptor, phage reversible adsorption Sources: GOC:bm Definition: Process by which a bacteriophage, using its tail fibers, spikes or a baseplate component, initially recognizes and binds to its specific receptor on the host cell surface. This process is reversible and allows the release of a bacteriophage without affecting infection.